{
  "term_id": "GO:0034703",
  "gene": "UniProtKB:P48995",
  "term_label": "cation channel complex",
  "gene_symbol": "TRPC1",
  "gene_name": "Short transient receptor potential channel 1"
}